{
  "gene": "UniProtKB:Q7Z2H8",
  "gene_name": "Proton-coupled amino acid transporter 1",
  "term_id": "GO:0015187",
  "term_label": "glycine transmembrane transporter activity",
  "gene_symbol": "SLC36A1"
}